{
  "gene": "UniProtKB:A6NHQ4",
  "term_id": "UNKNOWN:0003",
  "term_label": "Unknown cellular component",
  "gene_symbol": "EPOP",
  "gene_name": "Elongin BC and Polycomb repressive complex 2-associated protein"
}